formation of appressorium germ tube hook structure [GO:0075029] (biological process) Also known as: formation of germ tube tip of symbiont on or near the exterior of host, formation of symbiont germ tube hook structure for appressorium development, symbiont germ tube hook structure formation on or near host, formation of symbiont germ tube hook structure on or near host Regulation: regulated by modulation of formation of symbiont germ tube hook structure for appressorium development [GO:0075030]; positively regulated by positive regulation of formation of symbiont germ tube hook structure for appressorium development [GO:0075031]; negatively regulated by negative regulation of formation of symbiont germ tube hook structure for appressorium development [GO:0075032] Relationships: is a type of formation of infection structure [GO:0075015]; is part of GO:0075025 Definition: The development of a swollen tip at the growing end of a symbiont spore which usually flattens against the host cell surface prior to appressorium formation. Sources: GOC:pamgo_curators